{
  "gene_name": "Centrosome-associated protein ALMS1",
  "gene": "UniProtKB:Q8TCU4",
  "term_id": "UNKNOWN:0001",
  "term_label": "Unknown molecular function",
  "gene_symbol": "ALMS1"
}